{
  "gene_name": "Ankyrin repeat domain-containing protein 7",
  "gene": "UniProtKB:Q92527",
  "term_label": "Unknown molecular function",
  "term_id": "UNKNOWN:0001",
  "gene_symbol": "ANKRD7"
}